15-hydroxyprostaglandin-I dehydrogenase (NADP+) activity [GO:0047033] (MF) Sources: EC:1.1.1.231, RHEA:21420 Definition: Catalysis of the reaction: NADP+ + prostaglandin I(2) = 15-dehydro-prostaglandin I(2) + H+ + NADPH. Also known as: (5Z,13E)-(15S)-6,9alpha-epoxy-11alpha,15-dihydroxyprosta-5,13-dienoate:NADP+ 15-oxidoreductase activity, NADP+-dependent PGI2-specific 15-hydroxyprostaglandin dehydrogenase activity, NADP-linked 15-hydroxyprostaglandin (prostacyclin) dehydrogenase activity, PG I2 dehydrogenase activity, prostacyclin dehydrogenase activity Relationships: is a type of oxidoreductase activity, acting on the CH-OH group of donors, NAD or NADP as acceptor [GO:0016616]